{
  "term_id": "GO:0032216",
  "gene_symbol": "PIGW",
  "gene": "UniProtKB:Q7Z7B1",
  "gene_name": "Phosphatidylinositol-glycan biosynthesis class W protein",
  "term_label": "glucosaminyl-phosphatidylinositol O-acyltransferase activity"
}